ventriculo bulbo valve formation [GO:0003196] (biological process) Definition: The developmental process pertaining to the initial formation of the ventriculo bulbo valve from unspecified parts. This process begins with the specific processes that contribute to the appearance of the discrete structure and ends when the structural rudiment is recognizable. Sources: GOC:mtg_heart Relationships: is a type of heart valve formation [GO:0003188]; is part of ventriculo bulbo valve morphogenesis [GO:0003187]